response to host [GO:0075136] (biological process) Subtypes: symbiont-mediated response to host defenses [GO:0052200], response to host osmotic environment [GO:0075000], response to host redox environment [GO:0075137], GO:0075138, response to host iron concentration [GO:0075139], response to host pH environment [GO:0075293] Definition: Any process that results in a change in state or activity of the symbiont or its cell (in terms of movement, secretion, enzyme production, gene expression, etc.) as a result of detecting molecules of its host organism. The host is defined as the larger of the organisms involved in a symbiotic interaction. Sources: GOC:pamgo_curators Relationships: is a type of biological process involved in interaction with host [GO:0051701]; is a type of response to other organism [GO:0051707] Also known as: response of symbiont to host Note: Note that this term is used to annotate gene products of the symbiont.